{
  "gene_symbol": "GBA3",
  "term_id": "GO:0005829",
  "gene": "UniProtKB:Q9H227",
  "term_label": "cytosol",
  "gene_name": "Cytosolic beta-glucosidase"
}